{
  "gene_name": "Putative tripartite motif-containing protein 64B",
  "gene_symbol": "TRIM64B",
  "gene": "UniProtKB:A6NI03",
  "term_id": "GO:0061630",
  "term_label": "ubiquitin protein ligase activity"
}